posterior cell cortex [GO:0061803] (cellular component) Relationships: is a type of cell cortex region [GO:0099738] Definition: The region that lies just beneath the plasma membrane in the part of a cell that is closest to the posterior as defined by the developing, or existing, anterior/posterior axis. References: PMID:15666355, PMID:17981131 Sources: GOC:dph, GOC:kmv